intercalary heterochromatin [GO:0005725] (cellular component) Definition: Any of the regions of heterochromatin that form a reproducible set of dense bands scattered along the euchromatic arms in polytene chromosomes. References: PMID:14579245 Relationships: is_a GO:0000792